{
  "term_label": "mitochondrion",
  "term_id": "GO:0005739",
  "gene": "UniProtKB:Q9BXF6",
  "gene_symbol": "RAB11FIP5",
  "gene_name": "Rab11 family-interacting protein 5"
}